octopamine secretion, neurotransmission [GO:0061540] (BP) Sources: GOC:dph Definition: The controlled release of octopamine by a cell, in which the octopamine acts as a neurotransmitter. Relationships: is a type of neurotransmitter secretion [GO:0007269]; is a type of GO:0061539